{
  "gene_name": "Nucleolar and coiled-body phosphoprotein 1",
  "gene_symbol": "NOLC1",
  "term_label": "Unknown biological process",
  "term_id": "UNKNOWN:0002",
  "gene": "UniProtKB:Q14978"
}